{
  "gene_symbol": "NLE1",
  "term_id": "GO:0005730",
  "gene_name": "Notchless protein homolog 1",
  "gene": "UniProtKB:Q9NVX2",
  "term_label": "nucleolus"
}